{
  "gene_symbol": "C19orf12",
  "term_id": "UNKNOWN:0001",
  "gene": "UniProtKB:Q9NSK7",
  "gene_name": "Protein C19orf12",
  "term_label": "Unknown molecular function"
}